{
  "term_label": "regulation of intracellular signal transduction",
  "gene": "UniProtKB:O95379",
  "gene_name": "Tumor necrosis factor alpha-induced protein 8",
  "gene_symbol": "TNFAIP8",
  "term_id": "GO:1902531"
}